purine nucleobase binding [GO:0002060] (molecular function) Subtypes: adenine binding [GO:0002055], GO:0002057, xanthine binding [GO:0160050] Relationships: is a type of nucleobase binding [GO:0002054] Sources: GOC:hjd Definition: Binding to a purine nucleobase, an organic nitrogenous base with a purine skeleton. Also known as: purine base binding, purine binding